antigen processing and presentation of endogenous peptide antigen [GO:0002483] (biological process) Sources: GOC:add, ISBN:0781735149 Also known as: endogenous peptide antigen processing and presentation Definition: The process in which an antigen-presenting cell expresses a peptide antigen of endogenous origin on its cell surface in association with an MHC protein complex. The peptide is typically a fragment of a larger endogenous protein which has been degraded within the cell. Subtypes: antigen processing and presentation of endogenous peptide antigen via MHC class Ib [GO:0002476], antigen processing and presentation of endogenous peptide antigen via MHC class II [GO:0002491], antigen processing and presentation of endogenous peptide antigen via MHC class I [GO:0019885] Relationships: is a type of antigen processing and presentation of endogenous antigen [GO:0019883]; is a type of antigen processing and presentation of peptide antigen [GO:0048002]